inositol-5-diphosphate-1,3,4,6-tetrakisphosphate diphosphatase activity [GO:0106211] (molecular function) References: PMID:29540476 Sources: GOC:rn Definition: Catalysis of the reaction: 5-diphospho-1D-myo-inositol 1,3,4,6-tetrakisphosphate + H2O = 1D-myo-inositol 1,3,4,5,6-pentakisphosphate + H+ + phosphate. Relationships: is a type of inositol diphosphate tetrakisphosphate diphosphatase activity [GO:0052840] Also known as: 5-PP-InsP4 activity, 5-diphospho-myo-inositol 1,3,4,6-tetrakisphosphate diphosphatase activity, 5-diphosphoinositol 1,3,4,6-tetrakisphosphate diphosphatase activity